{
  "term_label": "Unknown biological process",
  "term_id": "UNKNOWN:0002",
  "gene": "UniProtKB:Q6ZUT4",
  "gene_name": "Putative uncharacterized protein FLJ43343",
  "gene_symbol": "Q6ZUT4"
}